5'-3' DNA exonuclease activity [GO:0035312] (molecular function) Subtypes: GO:0045145, double-stranded DNA 5'-3' DNA exonuclease activity [GO:0051908] Definition: Catalysis of the sequential cleavage of mononucleotides from a free 5' terminus of a DNA molecule. Relationships: is a type of 5'-3' exonuclease activity [GO:0008409]; is a type of DNA exonuclease activity, producing 5'-phosphomonoesters [GO:0016895] Also known as: 5'-3' exodeoxyribonuclease activity Sources: ISBN:0198547684